positive regulation of fatty acid metabolic process [GO:0045923] (biological process) Sources: GOC:go_curators Relationships: is a type of regulation of fatty acid metabolic process [GO:0019217]; is a type of positive regulation of lipid metabolic process [GO:0045834]; is a type of GO:0062013; positively regulates fatty acid metabolic process [GO:0006631] Also known as: positive regulation of fatty acid metabolism, up regulation of fatty acid metabolic process, up-regulation of fatty acid metabolic process, upregulation of fatty acid metabolic process, activation of fatty acid metabolic process, stimulation of fatty acid metabolic process Subtypes: positive regulation of fatty acid biosynthetic process [GO:0045723], positive regulation of fatty acid oxidation [GO:0046321], positive regulation of palmitic acid catabolic process [GO:0106395], positive regulation of methane biosynthetic process from 3-(methylthio)propionic acid [GO:1900335], positive regulation of butyryl-CoA catabolic process to butanol [GO:1900499] Definition: Any process that activates or increases the frequency, rate or extent of the chemical reactions and pathways involving fatty acids.